{
  "term_id": "GO:0043122",
  "term_label": "regulation of canonical NF-kappaB signal transduction",
  "gene_symbol": "PPM1B",
  "gene_name": "Protein phosphatase 1B",
  "gene": "UniProtKB:O75688"
}